{
  "term_label": "positive regulation of transcription by RNA polymerase II",
  "gene_name": "Thyroid hormone receptor beta",
  "gene_symbol": "THRB",
  "term_id": "GO:0045944",
  "gene": "UniProtKB:P10828"
}